{
  "gene_symbol": "CYSLTR2",
  "term_label": "cysteinyl leukotriene receptor activity",
  "gene": "UniProtKB:Q9NS75",
  "term_id": "GO:0001631",
  "gene_name": "Cysteinyl leukotriene receptor 2"
}